{
  "gene_name": "72 kDa type IV collagenase",
  "gene": "UniProtKB:P08253",
  "gene_symbol": "MMP2",
  "term_label": "tissue remodeling",
  "term_id": "GO:0048771"
}